{
  "gene": "UniProtKB:Q15825",
  "gene_name": "Neuronal acetylcholine receptor subunit alpha-6",
  "term_id": "GO:0005892",
  "term_label": "acetylcholine-gated channel complex",
  "gene_symbol": "CHRNA6"
}